{
  "gene": "UniProtKB:Q9BZA8",
  "term_label": "cell adhesion molecule binding",
  "gene_symbol": "PCDH11Y",
  "gene_name": "Protocadherin-11 Y-linked",
  "term_id": "GO:0050839"
}